{
  "term_label": "plasma membrane",
  "gene": "UniProtKB:P40198",
  "gene_symbol": "CEACAM3",
  "term_id": "GO:0005886",
  "gene_name": "Carcinoembryonic antigen-related cell adhesion molecule 3"
}